{
  "term_id": "UNKNOWN:0003",
  "gene_symbol": "IDNK",
  "term_label": "Unknown cellular component",
  "gene_name": "Probable gluconokinase",
  "gene": "UniProtKB:Q5T6J7"
}